{
  "term_label": "Unknown cellular component",
  "gene_symbol": "ANKRD66",
  "gene_name": "Ankyrin repeat domain-containing protein 66",
  "term_id": "UNKNOWN:0003",
  "gene": "UniProtKB:B4E2M5"
}